{
  "gene": "UniProtKB:Q9UNX9",
  "term_id": "GO:1990573",
  "term_label": "potassium ion import across plasma membrane",
  "gene_name": "ATP-sensitive inward rectifier potassium channel 14",
  "gene_symbol": "KCNJ14"
}